pectinesterase activity [GO:0030599] (molecular function) Definition: Catalysis of the reaction: pectin + n H2O = n methanol + pectate. Sources: EC:3.1.1.11 Also known as: pectin methylesterase activity, pectase activity, pectin demethoxylase activity, pectin methoxylase activity, pectin methyl esterase activity, pectin pectylhydrolase activity, pectinoesterase activity Relationships: is a type of carboxylic ester hydrolase activity [GO:0052689] Regulation: negatively regulated by pectinesterase inhibitor activity [GO:0046910]